{
  "gene": "UniProtKB:Q1ZZU3",
  "term_label": "Unknown molecular function",
  "gene_symbol": "SWI5",
  "gene_name": "DNA repair protein SWI5 homolog",
  "term_id": "UNKNOWN:0001"
}